{
  "term_id": "GO:0007160",
  "gene_name": "FRAS1-related extracellular matrix protein 2",
  "term_label": "cell-matrix adhesion",
  "gene_symbol": "FREM2",
  "gene": "UniProtKB:Q5SZK8"
}